{
  "gene_symbol": "ACP1",
  "term_label": "Unknown cellular component",
  "gene": "UniProtKB:P24666",
  "term_id": "UNKNOWN:0003",
  "gene_name": "Low molecular weight phosphotyrosine protein phosphatase"
}